{
  "gene": "UniProtKB:A5X5Y0",
  "term_id": "GO:0022850",
  "gene_symbol": "HTR3E",
  "gene_name": "5-hydroxytryptamine receptor 3E",
  "term_label": "serotonin-gated monoatomic cation channel activity"
}